{
  "gene_symbol": "SYT1",
  "gene_name": "Synaptotagmin-1",
  "term_label": "SNARE binding",
  "gene": "UniProtKB:P21579",
  "term_id": "GO:0000149"
}